{
  "gene_symbol": "PPY",
  "term_id": "GO:0005615",
  "gene_name": "Pancreatic polypeptide prohormone",
  "term_label": "extracellular space",
  "gene": "UniProtKB:P01298"
}